negative regulation of peptidyl-tyrosine phosphorylation [GO:0050732] (biological process) Relationships: is a type of negative regulation of protein phosphorylation [GO:0001933]; is a type of regulation of peptidyl-tyrosine phosphorylation [GO:0050730]; negatively regulates peptidyl-tyrosine phosphorylation [GO:0018108] Sources: GOC:ai Subtypes: negative regulation of tyrosine phosphorylation of STAT protein [GO:0042532], GO:0061099, negative regulation of peptidyl-tyrosine autophosphorylation [GO:1900085] Definition: Any process that stops, prevents, or reduces the frequency, rate or extent of the phosphorylation of peptidyl-tyrosine. Also known as: down regulation of peptidyl-tyrosine phosphorylation, down-regulation of peptidyl-tyrosine phosphorylation, downregulation of peptidyl-tyrosine phosphorylation, inhibition of peptidyl-tyrosine phosphorylation